amino sugar metabolic process [GO:0006040] (biological process) Sources: GOC:jl, ISBN:0192801023 Also known as: amino sugar metabolism, aminosaccharide metabolic process, aminosaccharide metabolism Subtypes: chitin metabolic process [GO:0006030], GO:0006041, N-acetylglucosamine metabolic process [GO:0006044], UDP-N-acetylglucosamine metabolic process [GO:0006047], N-acetylmannosamine metabolic process [GO:0006051], N-acetylneuraminate metabolic process [GO:0006054], UDP-N-acetylgalactosamine metabolic process [GO:0019276], fructosamine metabolic process [GO:0030389], amino sugar catabolic process [GO:0046348], amino sugar biosynthetic process [GO:0046349], lipid X metabolic process [GO:2001289] Definition: The chemical reactions and pathways involving any amino sugar, sugars containing an amino group in place of a hydroxyl group. Relationships: is_a carbohydrate derivative metabolic process [GO:1901135]